{
  "gene_name": "Uncharacterized protein",
  "gene_symbol": "A0A8V8TND5",
  "term_label": "Unknown biological process",
  "gene": "UniProtKB:A0A8V8TND5",
  "term_id": "UNKNOWN:0002"
}